{
  "term_label": "GTP binding",
  "term_id": "GO:0005525",
  "gene_name": "Rho-related BTB domain-containing protein 1",
  "gene_symbol": "RHOBTB1",
  "gene": "UniProtKB:O94844"
}